{
  "gene_symbol": "KYNU",
  "gene": "UniProtKB:Q16719",
  "term_id": "GO:0030429",
  "term_label": "kynureninase activity",
  "gene_name": "Kynureninase"
}